smooth muscle derived foam cell differentiation [GO:0090078] (biological process) Definition: The process in which a smooth muscle cell acquires the specialized features of a foam cell. A foam cell is a type of cell containing lipids in small vacuoles and typically seen in atherosclerotic lesions, as well as other conditions. Sources: GOC:BHF, GOC:add, GOC:dph, GOC:tb Relationships: is a type of foam cell differentiation [GO:0090077]